{
  "gene_symbol": "PLXNB1",
  "gene_name": "Plexin-B1",
  "term_label": "regulation of cell shape",
  "gene": "UniProtKB:O43157",
  "term_id": "GO:0008360"
}